{
  "gene_symbol": "TNRC6B",
  "term_label": "nucleoplasm",
  "gene": "UniProtKB:Q9UPQ9",
  "term_id": "GO:0005654",
  "gene_name": "Trinucleotide repeat-containing gene 6B protein"
}